{
  "gene_symbol": "KRTAP4-4",
  "term_label": "Unknown cellular component",
  "gene": "UniProtKB:Q9BYR3",
  "term_id": "UNKNOWN:0003",
  "gene_name": "Keratin-associated protein 4-4"
}